{
  "term_label": "regulation of cell migration",
  "gene_symbol": "PLXNA1",
  "term_id": "GO:0030334",
  "gene_name": "Plexin-A1",
  "gene": "UniProtKB:Q9UIW2"
}